histone H2AXS139 kinase activity [GO:0035979] (molecular function) Note: Note that the residue position corresponds to the canonical human H2AX histone (UniProtKB:P16104); this residue is conserved across all eukaryotes. Residue 1 is the first residue following removal of the initiating Methionine (Met). Note that each histone is encoded by multiple genes, and sequences may vary across different genes within an organism. Definition: Catalysis of the reaction: histone H2AX-serine (position 139) + ATP = histone H2AX-phosphoserine (position 139) + ADP. This reaction is the addition of a phosphate group to the serine residue at position 139 of histone variant H2AX. References: PMID:11893489, PMID:16061642 Relationships: is a type of protein serine/threonine kinase activity [GO:0004674]; is a type of GO:0141003 Also known as: histone kinase activity (H2A.x-S139 specific), histone H2AS139 kinase activity, histone kinase activity (H2A-S139 specific)